{
  "gene": "UniProtKB:Q8IYB1",
  "term_id": "UNKNOWN:0002",
  "gene_name": "Nucleotidyltransferase MB21D2",
  "term_label": "Unknown biological process",
  "gene_symbol": "MB21D2"
}